exo-1,4-beta-D-glucosaminidase activity [GO:0052761] (molecular function) Relationships: is a type of hydrolase activity, hydrolyzing O-glycosyl compounds [GO:0004553] Sources: EC:3.2.1.165, GOC:mengo_curators, MetaCyc:3.2.1.165-RXN Definition: Catalysis of the reaction: [beta-(1->4)-D-glucosamine]n-[N-acetyl-D-glucosamine]m = D-glucosamine + [beta-(1->4)-D-glucosamine](n-1)-[N-acetyl-D-glucosamine]m. This reaction is the hydrolysis of chitosan or chitosan oligosaccharides to remove a D-glucosamine residue from the non-reducing termini; chitosan is a linear polysaccharide composed of randomly distributed beta-(1->4)-linked D-glucosamine and N-acetyl-D-glucosamine units. Also known as: chitosan exo-1,4-beta-D-glucosaminidase activity, chitosan glucosaminohydrolase activity, exo-beta-D-glucosaminidase activity, exochitosanase activity